signal release [GO:0023061] (biological process) Definition: The process in which a signal is secreted or discharged into the extracellular medium from a cellular source. Also known as: signal secretion Sources: GOC:mtg_signal Relationships: is a type of GO:0032940; is part of cell-cell signaling [GO:0007267] Subtypes: serotonin secretion [GO:0001820], renin secretion into blood stream [GO:0002001], dopamine secretion [GO:0014046], prostaglandin secretion [GO:0032310], BMP secretion [GO:0038055], hormone secretion [GO:0046879], GO:0048243, Wnt protein secretion [GO:0061355], acetylcholine secretion [GO:0061526], signal release from synapse [GO:0099643]